{
  "gene_symbol": "CAMK2G",
  "gene_name": "Calcium_calmodulin-dependent protein kinase type II subunit gamma",
  "term_label": "regulation of neuron projection development",
  "term_id": "GO:0010975",
  "gene": "UniProtKB:Q13555"
}